{
  "gene": "UniProtKB:Q9Y4R7",
  "gene_name": "Tubulin monoglycylase TTLL3",
  "term_label": "sperm flagellum",
  "term_id": "GO:0036126",
  "gene_symbol": "TTLL3"
}